glycogen metabolic process [GO:0005977] (biological process) Definition: The chemical reactions and pathways involving glycogen, a polydisperse, highly branched glucan composed of chains of D-glucose residues in alpha-(1->4) glycosidic linkage, joined together by alpha-(1->6) glycosidic linkages. Sources: ISBN:0198506732 Also known as: glycogen metabolism Relationships: is a type of GO:0006112; is a type of glucan metabolic process [GO:0044042] Subtypes: GO:0005978, glycogen catabolic process [GO:0005980] Regulation: regulated by regulation of glycogen metabolic process [GO:0070873]; negatively regulated by negative regulation of glycogen metabolic process [GO:0070874]; positively regulated by GO:0070875